{
  "gene_name": "Interleukin-22 receptor subunit alpha-2",
  "gene": "UniProtKB:Q969J5",
  "term_id": "GO:0005886",
  "gene_symbol": "IL22RA2",
  "term_label": "plasma membrane"
}